regulation of synaptic assembly at neuromuscular junction [GO:0008582] (biological process) Sources: GOC:go_curators Relationships: is a type of regulation of developmental growth [GO:0048638]; is a type of regulation of synapse assembly [GO:0051963]; is a type of regulation of neuromuscular junction development [GO:1904396]; regulates synaptic assembly at neuromuscular junction [GO:0051124] Also known as: regulation of synaptic growth at neuromuscular junction Definition: Any process that modulates the frequency, rate or extent of synaptic assembly at neuromuscular junctions. Subtypes: negative regulation of synaptic assembly at neuromuscular junction [GO:0045886], positive regulation of synaptic assembly at neuromuscular junction [GO:0045887]